{
  "gene": "UniProtKB:Q8TAU0",
  "gene_name": "Homeobox protein Nkx-2.3",
  "term_label": "regulation of transcription by RNA polymerase II",
  "term_id": "GO:0006357",
  "gene_symbol": "NKX2-3"
}